{
  "term_label": "Unknown molecular function",
  "gene": "UniProtKB:Q9BSJ6",
  "gene_name": "Protein PIMREG",
  "gene_symbol": "PIMREG",
  "term_id": "UNKNOWN:0001"
}